clearance of foreign intracellular DNA [GO:0044355] (biological process) Definition: A defense process that protects an organism from invading foreign DNA. Relationships: is a type of GO:0099046 Subtypes: GO:0009307 Also known as: clearance of foreign intracellular DNA by conversion of DNA cytidine to uridine References: PMID:20062055 Sources: GO:jl